{
  "gene_symbol": "PGK2",
  "gene": "UniProtKB:P07205",
  "gene_name": "Phosphoglycerate kinase 2",
  "term_label": "phosphoglycerate kinase activity",
  "term_id": "GO:0004618"
}